{
  "gene_symbol": "SLC4A1",
  "gene_name": "Band 3 anion transport protein",
  "gene": "UniProtKB:P02730",
  "term_label": "transmembrane transport",
  "term_id": "GO:0055085"
}